negative regulation of GTPase activity [GO:0034260] (BP) Note: An example of this is P2xA in Dictyostelium (UniProt symbol Q86JM7) in PMID:24335649. Definition: Any process that stops or reduces the rate of GTP hydrolysis by a GTPase. Relationships: is a type of regulation of GTPase activity [GO:0043087]; is a type of GO:0048519; is a type of GO:0051346; negatively regulates GTPase activity [GO:0003924] References: PMID:16143306, PMID:24335649 Sources: GOC:TermGenie, GOC:mah, GOC:rb, GO_REF:0000058 Also known as: down regulation of GTPase activity, down-regulation of GTPase activity, downregulation of GTPase activity, negative regulation of guanosinetriphosphatase activity, down regulation of Rab GTPase activity, down regulation of Ras GTPase activity, down regulation of Rho GTPase activity, down regulation of regulation of Ran GTPase activity, down-regulation of Rab GTPase activity, down-regulation of Ras GTPase activity, down-regulation of Rho GTPase activity, down-regulation of regulation of Ran GTPase activity, downregulation of Rab GTPase activity, downregulation of Ras GTPase activity, downregulation of Rho GTPase activity, downregulation of regulation of Ran GTPase activity, inhibition of GTPase activity, inhibition of Rab GTPase activity, inhibition of Ras GTPase activity, inhibition of Rho GTPase activity, inhibition of regulation of Ran GTPase activity, negative regulation of Rab GTPase activity, negative regulation of Ran GTPase activity, negative regulation of Ras GTPase activity, negative regulation of Rho GTPase activity